{
  "gene_name": "Trifunctional purine biosynthetic protein adenosine-3",
  "term_label": "adenine biosynthetic process",
  "gene": "UniProtKB:P22102",
  "term_id": "GO:0046084",
  "gene_symbol": "GART"
}